{
  "term_id": "GO:0005737",
  "gene_symbol": "FOXRED1",
  "gene": "UniProtKB:Q96CU9",
  "term_label": "cytoplasm",
  "gene_name": "FAD-dependent oxidoreductase domain-containing protein 1"
}